{
  "gene": "UniProtKB:Q8NH90",
  "gene_symbol": "OR5AK2",
  "gene_name": "Olfactory receptor 5AK2",
  "term_label": "olfactory receptor activity",
  "term_id": "GO:0004984"
}